metallochaperone complex [GO:1902695] (cellular component) Definition: A protein complex which is capable of metallochaperone activity. References: PMID:10426947 Sources: GOC:TermGenie, GOC:bhm, GO_REF:0000088 Relationships: is a type of protein-containing complex [GO:0032991] Subtypes: superoxide dismutase copper chaperone complex [GO:1902694]